{
  "gene_name": "Heat shock factor protein 2",
  "gene": "UniProtKB:Q03933",
  "term_id": "GO:0000978",
  "term_label": "RNA polymerase II cis-regulatory region sequence-specific DNA binding",
  "gene_symbol": "HSF2"
}